{
  "gene": "UniProtKB:A0A0C4DH26",
  "gene_symbol": "IGKV6D-41",
  "term_label": "immune response",
  "gene_name": "Probable non-functional immunoglobulin kappa variable 6D-41",
  "term_id": "GO:0006955"
}